chronic inflammatory response to antigenic stimulus [GO:0002439] (biological process) Relationships: is a type of inflammatory response to antigenic stimulus [GO:0002437]; is a type of GO:0002544 Definition: A chronic inflammatory response to an antigenic stimulus. A chronic inflammatory response persists indefinitely during days, weeks, or months in the life of an individual. Regulation: regulated by regulation of chronic inflammatory response to antigenic stimulus [GO:0002874]; negatively regulated by GO:0002875; positively regulated by GO:0002876 Sources: GOC:add, ISBN:0781735149